{
  "term_id": "GO:0006357",
  "gene_symbol": "FOXJ1",
  "gene": "UniProtKB:Q92949",
  "term_label": "regulation of transcription by RNA polymerase II",
  "gene_name": "Forkhead box protein J1"
}